plastid single-subunit type RNA polymerase binding [GO:0001051] (MF) Relationships: is a type of single-subunit type RNA polymerase binding [GO:0001050] Definition: Binding to a single subunit plastid RNA polymerase enzyme, which is composed of a single catalytic subunit similar to the RNA polymerase enzymes from phages T3, T7, and SP6. References: PMID:20701995 Sources: GOC:txnOH